{
  "gene": "UniProtKB:Q6N075",
  "term_label": "Unknown molecular function",
  "gene_name": "Molybdate-anion transporter",
  "term_id": "UNKNOWN:0001",
  "gene_symbol": "MFSD5"
}